regulation of actin cortical patch localization [GO:0060583] (biological process) Relationships: is a type of regulation of cellular localization [GO:0060341]; regulates actin cortical patch localization [GO:0051666] Also known as: regulation of actin cortical patch localisation Sources: GOC:dph, GOC:tb Definition: Any process that modulates the localization of an actin cortical patch. An actin cortical patch is a discrete actin-containing structure found just beneath the plasma membrane in fungal cells.